{
  "term_label": "proton-transporting ATPase activity, rotational mechanism",
  "gene_symbol": "ATP6V1C2",
  "gene_name": "V-type proton ATPase subunit C 2",
  "term_id": "GO:0046961",
  "gene": "UniProtKB:Q8NEY4"
}